{
  "term_label": "heart contraction",
  "gene_name": "Myosin regulatory light chain 2, atrial isoform",
  "gene": "UniProtKB:Q01449",
  "term_id": "GO:0060047",
  "gene_symbol": "MYL7"
}